{
  "term_id": "GO:0070382",
  "gene": "UniProtKB:Q8NBV8",
  "gene_symbol": "SYT8",
  "term_label": "exocytic vesicle",
  "gene_name": "Synaptotagmin-8"
}